{
  "gene": "UniProtKB:Q3ZCM7",
  "term_id": "GO:0000226",
  "gene_name": "Tubulin beta-8 chain",
  "term_label": "microtubule cytoskeleton organization",
  "gene_symbol": "TUBB8"
}